{
  "term_id": "GO:0051924",
  "term_label": "regulation of calcium ion transport",
  "gene_name": "Extracellular calcium-sensing receptor",
  "gene_symbol": "CASR",
  "gene": "UniProtKB:P41180"
}